{
  "term_id": "GO:0031032",
  "gene": "UniProtKB:O43491",
  "gene_name": "Band 4.1-like protein 2",
  "term_label": "actomyosin structure organization",
  "gene_symbol": "EPB41L2"
}